{
  "term_label": "3',5'-cyclic-GMP phosphodiesterase activity",
  "gene_name": "cAMP-specific 3',5'-cyclic phosphodiesterase 4B",
  "gene_symbol": "PDE4B",
  "gene": "UniProtKB:Q07343",
  "term_id": "GO:0047555"
}